{
  "gene_name": "tRNA-specific adenosine deaminase 1",
  "gene": "UniProtKB:Q9BUB4",
  "gene_symbol": "ADAT1",
  "term_id": "GO:0008033",
  "term_label": "tRNA processing"
}